{
  "term_label": "plasma membrane",
  "gene_symbol": "SPHK1",
  "gene": "UniProtKB:Q9NYA1",
  "gene_name": "Sphingosine kinase 1",
  "term_id": "GO:0005886"
}